{
  "term_id": "GO:0006890",
  "term_label": "retrograde vesicle-mediated transport, Golgi to endoplasmic reticulum",
  "gene_name": "Coatomer subunit beta'",
  "gene": "UniProtKB:P35606",
  "gene_symbol": "COPB2"
}